{
  "term_label": "nickel cation transmembrane transporter activity",
  "gene_name": "Natural resistance-associated macrophage protein 2",
  "term_id": "GO:0015099",
  "gene": "UniProtKB:P49281",
  "gene_symbol": "SLC11A2"
}